response to desiccation [GO:0009269] (biological process) Sources: GOC:jl Subtypes: cellular response to desiccation [GO:0071465] Definition: Any process that results in a change in state or activity of a cell or an organism (in terms of movement, secretion, enzyme production, gene expression, etc.) as a result of a desiccation stimulus, extreme dryness resulting from the prolonged deprivation of water. Also known as: desiccation tolerance Relationships: is a type of response to water deprivation [GO:0009414]